{
  "gene_name": "Inositol hexakisphosphate kinase 1",
  "gene": "UniProtKB:Q92551",
  "gene_symbol": "IP6K1",
  "term_label": "nucleus",
  "term_id": "GO:0005634"
}